regulation of telomere maintenance via semi-conservative replication [GO:0032213] (biological process) Subtypes: negative regulation of telomere maintenance via semi-conservative replication [GO:0032214], GO:0032215 Definition: Any process that modulates the frequency, rate or extent of the semi-conservative replication of telomeric DNA. Relationships: is a type of regulation of cell cycle process [GO:0010564]; is a type of regulation of telomere maintenance [GO:0032204]; regulates telomere maintenance via semi-conservative replication [GO:0032201] Sources: GOC:mah